{
  "gene_symbol": "POTEG",
  "gene_name": "POTE ankyrin domain family member G",
  "term_id": "UNKNOWN:0002",
  "gene": "UniProtKB:Q6S5H5",
  "term_label": "Unknown biological process"
}